{
  "term_label": "aspartic endopeptidase activity, intramembrane cleaving",
  "gene": "UniProtKB:Q8TCT9",
  "gene_symbol": "HM13",
  "gene_name": "Minor histocompatibility antigen H13",
  "term_id": "GO:0042500"
}